{
  "gene": "UniProtKB:Q06609",
  "gene_symbol": "RAD51",
  "term_label": "mitotic recombination",
  "term_id": "GO:0006312",
  "gene_name": "DNA repair protein RAD51 homolog 1"
}